2-iminopropanoate deaminase activity [GO:0120243] (MF) Also known as: 2-iminobutanoate/2-iminopropanoate deaminase Sources: RHEA:40671 Relationships: is a type of 2-iminobutanoate/2-iminopropanoate deaminase [GO:0120241] Definition: Catalysis of the reaction: 2-iminopropanoate + H2O = NH4(+) + pyruvate.